{
  "gene_name": "Golgi SNAP receptor complex member 1",
  "term_id": "GO:0000139",
  "term_label": "Golgi membrane",
  "gene": "UniProtKB:O95249",
  "gene_symbol": "GOSR1"
}